{
  "term_id": "GO:0008239",
  "gene_name": "Dipeptidyl peptidase 4",
  "gene_symbol": "DPP4",
  "term_label": "dipeptidyl-peptidase activity",
  "gene": "UniProtKB:P27487"
}